nucleotide-excision repair involved in interstrand cross-link repair [GO:1901255] (BP) Relationships: is a type of GO:0006289; is part of interstrand cross-link repair [GO:0036297] References: PMID:22064477 Sources: GOC:TermGenie Also known as: NER involved in ICL repair, NER involved in interstrand cross-link repair, nucleotide-excision repair involved in ICL repair Definition: Any nucleotide-excision repair that is involved in interstrand cross-link repair.